red light signaling pathway [GO:0010161] (biological process) Relationships: is a type of red or far-red light signaling pathway [GO:0010017]; is a type of cellular response to red light [GO:0071491] Definition: The series of molecular signals initiated upon sensing of red light by a photoreceptor molecule. Red light is electromagnetic radiation of wavelength of 580-700nm. An example of this response is seen at the beginning of many plant species developmental stages. These include germination, and the point when cotyledon expansion is triggered. In certain species these processes take place in response to absorption of red light by the pigment molecule phytochrome, but the signal can be reversed by exposure to far red light. During the initial phase the phytochrome molecule is only present in the red light absorbing form, but on absorption of red light it changes to a far red light absorbing form, triggering progress through development. An immediate short period of exposure to far red light entirely returns the pigment to its initial state and prevents triggering of the developmental process. A thirty minute break between red and subsequent far red light exposure renders the red light effect irreversible, and development then occurs regardless of whether far red light exposure subsequently occurs. Sources: GOC:mtg_far_red, GOC:sm Also known as: red light phototransduction, red light signal transduction, red light signalling pathway